{
  "gene_symbol": "AOAH",
  "gene_name": "Acyloxyacyl hydrolase",
  "term_label": "Unknown cellular component",
  "term_id": "UNKNOWN:0003",
  "gene": "UniProtKB:P28039"
}